{
  "gene_name": "Leucine-rich repeat-containing protein 58",
  "gene": "UniProtKB:Q96CX6",
  "term_label": "Unknown molecular function",
  "term_id": "UNKNOWN:0001",
  "gene_symbol": "LRRC58"
}